protein demannosylation [GO:0036507] (BP) Note: Consider also annotating to the term 'mannosyl-oligosaccharide 1,2-alpha-mannosidase activity ; GO:0004571'. References: PMID:25092655 Sources: GOC:PARL, GOC:bf Also known as: protein de-mannosylation Subtypes: GO:0036508 Relationships: is a type of GO:0006517; has part mannosidase activity [GO:0015923] Definition: The removal of one or more mannose residues from a mannosylated protein.